{
  "term_label": "DNA-binding transcription factor activity, RNA polymerase II-specific",
  "gene": "UniProtKB:Q00577",
  "gene_name": "Transcriptional activator protein Pur-alpha",
  "term_id": "GO:0000981",
  "gene_symbol": "PURA"
}